{
  "term_label": "cytoplasm",
  "gene_symbol": "SRPK3",
  "gene": "UniProtKB:Q9UPE1",
  "gene_name": "SRSF protein kinase 3",
  "term_id": "GO:0005737"
}